{
  "term_label": "positive regulation of cell migration",
  "gene": "UniProtKB:O15444",
  "gene_name": "C-C motif chemokine 25",
  "term_id": "GO:0030335",
  "gene_symbol": "CCL25"
}